{
  "term_id": "GO:0005634",
  "gene_symbol": "EZH1",
  "gene_name": "Histone-lysine N-methyltransferase EZH1",
  "term_label": "nucleus",
  "gene": "UniProtKB:Q92800"
}